{
  "gene_name": "Mitotic interactor and substrate of PLK1",
  "term_label": "Unknown biological process",
  "gene": "UniProtKB:Q8IVT2",
  "term_id": "UNKNOWN:0002",
  "gene_symbol": "MISP"
}